{
  "gene_name": "Secernin-2",
  "gene_symbol": "SCRN2",
  "term_label": "Unknown biological process",
  "gene": "UniProtKB:Q96FV2",
  "term_id": "UNKNOWN:0002"
}